myoblast maturation [GO:0048628] (biological process) Sources: CL:0000056, GOC:dph, GOC:mtg_muscle Definition: A developmental process, independent of morphogenetic (shape) change, that is required for a myoblast to attain its fully functional state. A myoblast is a mononucleate cell type that, by fusion with other myoblasts, gives rise to the myotubes that eventually develop into skeletal muscle fibers. Relationships: is a type of cell maturation [GO:0048469]; is part of myoblast development [GO:0048627] Subtypes: myoblast maturation involved in muscle regeneration [GO:0014914]